{
  "gene": "UniProtKB:Q9P2E2",
  "gene_name": "Kinesin-like protein KIF17",
  "term_id": "GO:0008017",
  "term_label": "microtubule binding",
  "gene_symbol": "KIF17"
}